{
  "gene_symbol": "Q8TAT8",
  "term_label": "Unknown biological process",
  "gene_name": "Putative uncharacterized protein LOC644613",
  "term_id": "UNKNOWN:0002",
  "gene": "UniProtKB:Q8TAT8"
}